{
  "gene_name": "Putative speedy protein-like protein 3",
  "gene": "UniProtKB:A6NJR5",
  "term_label": "Unknown cellular component",
  "gene_symbol": "A6NJR5",
  "term_id": "UNKNOWN:0003"
}